positive regulation of adenylate cyclase-activating G protein-coupled receptor signaling pathway [GO:0106071] (biological process) Definition: Any process that activates or increases the frequency, rate or extent of an adenylate cyclase-activating G protein-coupled receptor signaling pathway. Also known as: positive regulation of adenylate cyclase-activating G-protein coupled receptor signaling pathway Relationships: is a type of positive regulation of G protein-coupled receptor signaling pathway [GO:0045745]; is a type of regulation of adenylate cyclase-activating G protein-coupled receptor signaling pathway [GO:0106070]; positively regulates adenylate cyclase-activating G protein-coupled receptor signaling pathway [GO:0007189] References: PMID:19246489 Sources: GOC:hjd Subtypes: positive regulation of adenylate cyclase-activating adrenergic receptor signaling pathway involved in heart process [GO:0140196]